perception of rate of movement [GO:0019232] (biological process) Definition: The series of events by which an organism senses the speed and direction of movement of the body and its parts. Sources: GOC:mah Also known as: kinesthesia Relationships: is a type of proprioception [GO:0019230]